{
  "term_id": "GO:0005385",
  "gene_symbol": "SLC30A2",
  "gene": "UniProtKB:Q9BRI3",
  "term_label": "zinc ion transmembrane transporter activity",
  "gene_name": "Proton-coupled zinc antiporter SLC30A2"
}